{
  "gene_symbol": "TAX1BP1",
  "term_label": "negative regulation of apoptotic process",
  "gene": "UniProtKB:Q86VP1",
  "gene_name": "Tax1-binding protein 1",
  "term_id": "GO:0043066"
}